{
  "gene_name": "Melanoma-associated antigen B6B",
  "gene": "UniProtKB:A0A0J9YX57",
  "term_label": "Unknown molecular function",
  "gene_symbol": "MAGEB6B",
  "term_id": "UNKNOWN:0001"
}